{
  "term_label": "phosphoprotein phosphatase activity",
  "term_id": "GO:0004721",
  "gene_symbol": "SSH3",
  "gene": "UniProtKB:Q8TE77",
  "gene_name": "Protein phosphatase Slingshot homolog 3"
}